{
  "gene_name": "Olfactory receptor 9Q2",
  "gene_symbol": "OR9Q2",
  "term_id": "GO:0005549",
  "term_label": "odorant binding",
  "gene": "UniProtKB:Q8NGE9"
}